M/G1 phase-specific MADS box-forkhead transcription factor complex [GO:0097221] (cellular component) Also known as: PBF complex, PBF transcription complex, PCB binding factor complex, pombe cell cycle box binding factor complex Definition: A protein complex that contains a MADS-box protein and two forkhead domain proteins, and binds to and regulates transcription from promoters of genes transcribed during the M/G1 transition of the cell cycle. In Schizosaccharomyces pombe, the complex contains the MADS-box protein Mbx1 and two forkhead proteins, Sep1 and Fkh2. References: PMID:18057023 Sources: GOC:mah Relationships: is a type of RNA polymerase II transcription regulator complex [GO:0090575]